{
  "term_label": "centrosome cycle",
  "gene_symbol": "PARD6A",
  "gene": "UniProtKB:Q9NPB6",
  "gene_name": "Partitioning defective 6 homolog alpha",
  "term_id": "GO:0007098"
}